{
  "gene": "UniProtKB:Q9GZU8",
  "term_id": "UNKNOWN:0001",
  "gene_name": "PSME3-interacting protein",
  "gene_symbol": "PSME3IP1",
  "term_label": "Unknown molecular function"
}